{
  "term_label": "G protein-coupled dopamine receptor signaling pathway",
  "gene_name": "Guanine nucleotide-binding protein subunit beta-5",
  "gene": "UniProtKB:O14775",
  "gene_symbol": "GNB5",
  "term_id": "GO:0007212"
}